{
  "term_id": "GO:0031410",
  "term_label": "cytoplasmic vesicle",
  "gene_symbol": "DENND4C",
  "gene": "UniProtKB:Q5VZ89",
  "gene_name": "DENN domain-containing protein 4C"
}